{
  "term_id": "GO:0030574",
  "term_label": "collagen catabolic process",
  "gene_symbol": "MMP10",
  "gene": "UniProtKB:P09238",
  "gene_name": "Stromelysin-2"
}